{
  "gene": "UniProtKB:O14772",
  "gene_symbol": "FPGT",
  "term_id": "UNKNOWN:0003",
  "gene_name": "Fucose-1-phosphate guanylyltransferase",
  "term_label": "Unknown cellular component"
}